regulation of aecium development [GO:0075268] (biological process) Relationships: is a type of regulation of reproductive fruiting body development [GO:0031155]; regulates aecium development [GO:0075267] Definition: Any process that modulates the frequency, rate or extent of aecium development, a process in which a cuplike structure containing chains of aeciospores is formed. Sources: GOC:pamgo_curators Subtypes: positive regulation of aecium development [GO:0075269], GO:0075270